{
  "gene_name": "Protein SOX-15",
  "term_label": "RNA polymerase II cis-regulatory region sequence-specific DNA binding",
  "gene": "UniProtKB:O60248",
  "term_id": "GO:0000978",
  "gene_symbol": "SOX15"
}